{
  "term_label": "synapse",
  "gene_name": "Protein sidekick-1",
  "term_id": "GO:0045202",
  "gene_symbol": "SDK1",
  "gene": "UniProtKB:Q7Z5N4"
}